tarsal gland development [GO:1903699] (biological process) References: PMID:20664693 Sources: GOC:TermGenie, GO_REF:0000094 Definition: The process whose specific outcome is the progression of a tarsal gland over time, from its formation to the mature structure. Also known as: Meibomian gland development, gland of Meibom development, glandula tarsales development, tarsoconjunctival gland development Relationships: is_a GO:0048733